{
  "term_id": "UNKNOWN:0001",
  "gene": "UniProtKB:Q9P1F3",
  "gene_name": "Costars family protein ABRACL",
  "term_label": "Unknown molecular function",
  "gene_symbol": "ABRACL"
}